{
  "gene_name": "Putative endoplasmin-like protein",
  "gene": "UniProtKB:Q58FF3",
  "term_id": "GO:0006457",
  "term_label": "protein folding",
  "gene_symbol": "HSP90B2P"
}